{
  "gene": "UniProtKB:Q9Y2H6",
  "gene_name": "Fibronectin type-III domain-containing protein 3A",
  "term_label": "Unknown molecular function",
  "gene_symbol": "FNDC3A",
  "term_id": "UNKNOWN:0001"
}